response to vitamin D [GO:0033280] (biological process) Relationships: is a type of GO:0033273; is a type of GO:0033993; is a type of response to oxygen-containing compound [GO:1901700] Also known as: response to calciferol, response to cholecalciferol, response to ergocalciferol Subtypes: cellular response to vitamin D [GO:0071305] Definition: Any process that results in a change in state or activity of a cell or an organism (in terms of movement, secretion, enzyme production, gene expression, etc.) as a result of a vitamin D stimulus. Sources: GOC:sl